{
  "gene_symbol": "DUX4L4",
  "gene_name": "Double homeobox protein 4-like protein 4",
  "term_id": "GO:0005634",
  "gene": "UniProtKB:P0CJ87",
  "term_label": "nucleus"
}